{
  "gene_symbol": "CD160",
  "term_label": "Unknown molecular function",
  "term_id": "UNKNOWN:0001",
  "gene_name": "CD160 antigen",
  "gene": "UniProtKB:O95971"
}